{
  "term_id": "UNKNOWN:0002",
  "gene_symbol": "HRURF",
  "gene": "UniProtKB:P0DUH7",
  "gene_name": "Protein HRURF",
  "term_label": "Unknown biological process"
}